{
  "gene": "UniProtKB:O60427",
  "gene_symbol": "FADS1",
  "term_label": "oxidoreductase activity, acting on paired donors, with oxidation of a pair of donors resulting in the reduction of molecular oxygen to two molecules of water",
  "gene_name": "Acyl-CoA (8-3)-desaturase",
  "term_id": "GO:0016717"
}